{
  "gene": "UniProtKB:P22090",
  "term_label": "cytosolic small ribosomal subunit",
  "gene_symbol": "RPS4Y1",
  "gene_name": "Small ribosomal subunit protein eS4, Y isoform 1",
  "term_id": "GO:0022627"
}